{
  "term_id": "UNKNOWN:0002",
  "gene_name": "Down syndrome critical region protein 10",
  "gene": "UniProtKB:P59022",
  "gene_symbol": "DSCR10",
  "term_label": "Unknown biological process"
}